positive regulation of protein activation cascade [GO:2000259] (biological process) Definition: Any process that activates or increases the frequency, rate or extent of protein activation cascade. Also known as: positive regulation of protein activation pathway, positive regulation of protein activitory cascade Subtypes: positive regulation of kinin cascade [GO:0002258], positive regulation of Toll receptor ligand protein activation cascade [GO:0160034], positive regulation of blood coagulation, common pathway [GO:2000262], positive regulation of blood coagulation, extrinsic pathway [GO:2000265], positive regulation of blood coagulation, intrinsic pathway [GO:2000268] Relationships: is a type of positive regulation of protein maturation [GO:1903319]; is a type of GO:2000257; positively regulates protein activation cascade [GO:0072376] Sources: GOC:mah